{
  "gene": "UniProtKB:P60903",
  "term_label": "cytoplasm",
  "gene_name": "Protein S100-A10",
  "gene_symbol": "S100A10",
  "term_id": "GO:0005737"
}